polaroplast [GO:0160201] (cellular component) References: PMID:16005007, PMID:19673893 Sources: Wikipedia:polaroplast Relationships: is_a intracellular membrane-bounded organelle [GO:0043231] Definition: A membrane-bounded organelle found in a microsporidian spore,  that swells with water, and exerts pressure to rupture the polar cap and evert the polar tube through which the sporoplasm escapes to infect the host.